{
  "term_label": "epidermis development",
  "gene_symbol": "SPINT1",
  "term_id": "GO:0008544",
  "gene_name": "Kunitz-type protease inhibitor 1",
  "gene": "UniProtKB:O43278"
}